{
  "term_id": "GO:0006597",
  "gene_symbol": "SMS",
  "gene": "UniProtKB:P52788",
  "term_label": "spermine biosynthetic process",
  "gene_name": "Spermine synthase"
}